{
  "gene": "UniProtKB:O95500",
  "term_id": "UNKNOWN:0001",
  "gene_symbol": "CLDN14",
  "gene_name": "Claudin-14",
  "term_label": "Unknown molecular function"
}